negative regulation of postsynaptic density assembly [GO:0160037] (biological process) References: PMID:17626212 Relationships: is_a regulation of postsynaptic density assembly [GO:0099151]; is a type of negative regulation of organelle assembly [GO:1902116]; is a type of negative regulation of postsynaptic density organization [GO:1905875]; negatively regulates postsynaptic density assembly [GO:0097107] Definition: Any process that decreases the rate, frequency, or extent of postsynaptic density assembly.